{
  "gene_name": "Actin-like protein 6A",
  "gene": "UniProtKB:O96019",
  "term_id": "GO:0016514",
  "gene_symbol": "ACTL6A",
  "term_label": "SWI/SNF complex"
}